chaperonin-containing T-complex [GO:0005832] (cellular component) Definition: A multisubunit ring-shaped complex that mediates protein folding in the cytosol without a cofactor. References: PMID:11580267 Sources: GOC:sgd_curators Relationships: is a type of protein folding chaperone complex [GO:0101031]; BFO_0000050 cytosol [GO:0005829] Also known as: CCT particle, TriC